tyramine receptor activity [GO:0008226] (molecular function) Definition: Combining with the biogenic amine tyramine to initiate a change in cell activity. Tyramine is a sympathomimetic amine derived from tyrosine with an action resembling that of epinephrine. Relationships: is a type of G protein-coupled amine receptor activity [GO:0008227] Sources: GOC:curators